{
  "gene": "UniProtKB:Q6QN14",
  "gene_name": "Ubiquitin carboxyl-terminal hydrolase 17-like protein 6",
  "term_label": "cysteine-type deubiquitinase activity",
  "gene_symbol": "USP17L6P",
  "term_id": "GO:0004843"
}